{
  "gene_symbol": "HSPB6",
  "gene": "UniProtKB:O14558",
  "gene_name": "Heat shock protein beta-6",
  "term_id": "GO:0043066",
  "term_label": "negative regulation of apoptotic process"
}